{
  "term_label": "serine-type endopeptidase activity",
  "term_id": "GO:0004252",
  "gene": "UniProtKB:Q6UWY2",
  "gene_symbol": "PRSS57",
  "gene_name": "Serine protease 57"
}